establishment of thoracic bristle planar orientation [GO:0048106] (biological process) Also known as: establishment of body bristle planar orientation Sources: FBbt:00004298, FBbt:00004408, GOC:ascb_2009, GOC:dph, GOC:jid Definition: Orientation along the body surface of bristles, sensory organs originating from a sensory organ precursor cell, such that they all point in a uniform direction. Relationships: is a type of GO:0048104; is part of chaeta morphogenesis [GO:0008407]